{
  "gene_name": "Sorting nexin-27",
  "term_id": "GO:0032456",
  "term_label": "endocytic recycling",
  "gene_symbol": "SNX27",
  "gene": "UniProtKB:Q96L92"
}